negative regulation of protein tyrosine kinase activity [GO:0061099] (biological process) Subtypes: negative regulation of epidermal growth factor-activated receptor activity [GO:0007175] Sources: GOC:dph, GOC:tb Definition: Any process that decreases the rate, frequency, or extent of protein tyrosine kinase activity. Relationships: is a type of negative regulation of protein kinase activity [GO:0006469]; is a type of negative regulation of peptidyl-tyrosine phosphorylation [GO:0050732]; is a type of regulation of protein tyrosine kinase activity [GO:0061097]; negatively regulates protein tyrosine kinase activity [GO:0004713]